protein serine/threonine phosphatase inhibitor activity [GO:0004865] (molecular function) Sources: GOC:dph, GOC:tb Definition: Binds to and stops, prevents or reduces the activity of a serine/threonine protein phosphatase, an enzyme that catalyzes the reaction: protein serine/threonine phosphate + H2O = protein serine/threonine + phosphate. Relationships: is a type of GO:0004864; negatively regulates GO:0004722